{
  "gene_name": "Proline-rich AKT1 substrate 1",
  "gene": "UniProtKB:Q96B36",
  "gene_symbol": "AKT1S1",
  "term_label": "Unknown molecular function",
  "term_id": "UNKNOWN:0001"
}